{
  "term_label": "ubiquitin-dependent protein catabolic process",
  "gene_name": "Probable E3 ubiquitin-protein ligase HERC6",
  "gene_symbol": "HERC6",
  "gene": "UniProtKB:Q8IVU3",
  "term_id": "GO:0006511"
}